{
  "gene": "UniProtKB:A6NK59",
  "gene_symbol": "ASB14",
  "term_label": "Unknown biological process",
  "gene_name": "Ankyrin repeat and SOCS box protein 14",
  "term_id": "UNKNOWN:0002"
}